trimethyllysine dioxygenase activity [GO:0050353] (molecular function) Sources: EC:1.14.11.8, RHEA:14181 Also known as: 6-N,6-N,6-N-trimethyl-L-lysine,2-oxoglutarate:oxygen oxidoreductase (3-hydroxylating), N6,N6,N6-trimethyl-L-lysine,2-oxoglutarate:oxygen oxidoreductase (3-hydroxylating), TML dioxygenase activity, TML hydroxylase activity, TML-alpha-ketoglutarate dioxygenase activity, TMLD activity, epsilon-trimethyllysine 2-oxoglutarate dioxygenase activity, trimethyllysine alpha-ketoglutarate dioxygenase activity, trimethyllysine,2-oxoglutarate dioxygenase activity Relationships: is a type of 2-oxoglutarate-dependent dioxygenase activity [GO:0016706] Definition: Catalysis of the reaction: 2-oxoglutarate + N(6),N(6),N(6)-trimethyl-L-lysine + O2 = 3-hydroxy-N(6),N(6),N(6)-trimethyl-L-lysine + CO2 + succinate.